{
  "gene": "UniProtKB:Q9ULI3",
  "term_label": "Unknown molecular function",
  "gene_symbol": "HEG1",
  "gene_name": "Protein HEG homolog 1",
  "term_id": "UNKNOWN:0001"
}